{
  "term_id": "GO:0005829",
  "gene_name": "Ubiquitin carboxyl-terminal hydrolase 48",
  "gene": "UniProtKB:Q86UV5",
  "term_label": "cytosol",
  "gene_symbol": "USP48"
}